{
  "term_label": "smoothened signaling pathway",
  "gene_symbol": "GLI1",
  "term_id": "GO:0007224",
  "gene_name": "Zinc finger protein GLI1",
  "gene": "UniProtKB:P08151"
}